{
  "gene_symbol": "MSH3",
  "gene": "UniProtKB:P20585",
  "term_id": "GO:0003690",
  "gene_name": "DNA mismatch repair protein Msh3",
  "term_label": "double-stranded DNA binding"
}